regulation of circadian sleep/wake cycle, sleep [GO:0045187] (biological process) Subtypes: regulation of circadian sleep/wake cycle, REM sleep [GO:0042320], GO:0042321, GO:0045188, positive regulation of circadian sleep/wake cycle, sleep [GO:0045938] Definition: Any process that modulates the frequency, rate or extent of sleep; a readily reversible state of reduced awareness and metabolic activity that occurs periodically in many animals. Relationships: is a type of regulation of circadian sleep/wake cycle [GO:0042749]; regulates GO:0050802 Sources: GOC:jl, ISBN:0192800981 Also known as: regulation of sleep